{
  "gene_symbol": "SPRTN",
  "term_label": "nucleus",
  "term_id": "GO:0005634",
  "gene": "UniProtKB:Q9H040",
  "gene_name": "DNA-dependent metalloprotease SPRTN"
}